{
  "term_id": "GO:0035613",
  "gene_symbol": "ERVK-8",
  "gene_name": "Endogenous retrovirus group K member 8 Pol protein",
  "gene": "UniProtKB:P63133",
  "term_label": "RNA stem-loop binding"
}